{
  "gene": "UniProtKB:Q9Y324",
  "term_label": "small-subunit processome",
  "gene_symbol": "FCF1",
  "term_id": "GO:0032040",
  "gene_name": "rRNA-processing protein FCF1 homolog"
}